{
  "term_id": "GO:0007165",
  "term_label": "signal transduction",
  "gene": "UniProtKB:P49593",
  "gene_name": "Protein phosphatase 1F",
  "gene_symbol": "PPM1F"
}